{
  "term_label": "RNA polymerase II, core complex",
  "gene": "UniProtKB:Q9GZM3",
  "gene_symbol": "POLR2J2",
  "gene_name": "DNA-directed RNA polymerase II subunit RPB11-b1",
  "term_id": "GO:0005665"
}